{
  "term_label": "calcium ion binding",
  "gene": "UniProtKB:P41208",
  "gene_name": "Centrin-2",
  "term_id": "GO:0005509",
  "gene_symbol": "CETN2"
}